{
  "gene_symbol": "IQCB1",
  "gene": "UniProtKB:Q15051",
  "gene_name": "IQ calmodulin-binding motif-containing protein 1",
  "term_label": "cilium",
  "term_id": "GO:0005929"
}